{
  "gene_symbol": "CES4A",
  "gene_name": "Carboxylesterase 4A",
  "term_id": "GO:0106435",
  "term_label": "carboxylesterase activity",
  "gene": "UniProtKB:Q5XG92"
}